{
  "gene": "UniProtKB:P41279",
  "term_label": "Unknown molecular function",
  "term_id": "UNKNOWN:0001",
  "gene_symbol": "MAP3K8",
  "gene_name": "Mitogen-activated protein kinase kinase kinase 8"
}